germline stem cell asymmetric division [GO:0098728] (biological process) Definition: The self-renewing division of a germline stem cell, to produce a daughter stem cell and a daughter germ cell which will divide to form one or more gametes. Sources: GOC:dos Relationships: is a type of germ-line stem cell division [GO:0042078]; is a type of asymmetric stem cell division [GO:0098722] Subtypes: female germ-line stem cell asymmetric division [GO:0048132], male germ-line stem cell asymmetric division [GO:0048133]